{
  "gene_symbol": "ACTB",
  "gene_name": "Actin, cytoplasmic 1",
  "term_id": "GO:0015629",
  "term_label": "actin cytoskeleton",
  "gene": "UniProtKB:P60709"
}